{
  "term_label": "actin filament binding",
  "gene": "UniProtKB:P06396",
  "gene_name": "Gelsolin",
  "term_id": "GO:0051015",
  "gene_symbol": "GSN"
}